5-hydroxyfuranocoumarin 5-O-methyltransferase activity [GO:0030752] (molecular function) Also known as: BMT activity, S-adenosyl-L-methionine:5-hydroxyfuranocoumarin 5-O-methyltransferase activity, S-adenosyl-L-methionine:5-hydroxyfurocoumarin 5-O-methyltransferase activity, S-adenosyl-L-methionine:bergaptol O-methyltransferase activity, S-adenosyl-L-methionine:bergaptolO-methyltransferase activity, bergaptol 5-O-methyltransferase activity, bergaptol O-methyltransferase activity, bergaptol methyltransferase activity, furanocoumarin 5-O-methyltransferase activity, furanocoumarin 5-methyltransferase activity Relationships: is a type of S-adenosylmethionine-dependent methyltransferase activity [GO:0008757] Sources: RHEA:18861 Definition: Catalysis of the reaction: a 5-hydroxyfurocoumarin + S-adenosyl-L-methionine = a 5-methoxyfurocoumarin + S-adenosyl-L-homocysteine + H+.